{
  "gene_name": "Exosome complex exonuclease RRP44",
  "gene_symbol": "DIS3",
  "term_label": "endonuclease activity",
  "term_id": "GO:0004519",
  "gene": "UniProtKB:Q9Y2L1"
}